{
  "gene_name": "RING finger protein 39",
  "gene": "UniProtKB:Q9H2S5",
  "term_label": "innate immune response",
  "gene_symbol": "RNF39",
  "term_id": "GO:0045087"
}